{
  "term_label": "nucleus",
  "gene_symbol": "NPLOC4",
  "term_id": "GO:0005634",
  "gene_name": "Nuclear protein localization protein 4 homolog",
  "gene": "UniProtKB:Q8TAT6"
}